{
  "term_id": "GO:0005643",
  "gene_name": "Nuclear pore complex protein Nup214",
  "term_label": "nuclear pore",
  "gene": "UniProtKB:P35658",
  "gene_symbol": "NUP214"
}